{
  "gene_name": "Melanoma-associated antigen F1",
  "term_label": "negative regulation of transcription by RNA polymerase II",
  "gene_symbol": "MAGEF1",
  "gene": "UniProtKB:Q9HAY2",
  "term_id": "GO:0000122"
}